Spemann organizer formation at the dorsal lip of the blastopore [GO:0060062] (biological process) Note: Occurs in amphibia, cephalochordates, cyclostomes and cartilaginous fish. Also known as: Spemann's organizer formation at the dorsal lip of the blastopore, Spemann-Mangold organizer formation at the dorsal lip of the blastopore Definition: Formation of the specialized region at the dorsal lip of the blatopore of the embryo that acts as the main signaling center establishing the vertebrate body plan. Relationships: is a type of Spemann organizer formation [GO:0060061] References: PMID:9442883 Sources: GOC:dph